symbiont-mediated disruption of host mucosa [GO:0141139] (BP) References: PMID:22520462, PMID:28598765, PMID:28764997 Definition: The disruption of the host mucosa by a symbiont, leading to damage or temporary subversion of that tissue. The mucosa is a membrane that lines various cavities in the body of an organism and covers the surface of internal organs. Relationships: is_a GO:0141146